collagen type XVII trimer [GO:0030937] (cellular component) Definition: A collagen homotrimer of alpha1(XVII) chains; type XVII collagen triple helices span the plasma membrane and associate with hemidesmosomes and the basal lamina where they bind laminin. Relationships: is a type of transmembrane collagen trimer [GO:0030936]; is a type of GO:0098637 References: PMID:19693541, PMID:21421911